pole plasm assembly [GO:0007315] (biological process) Sources: GOC:mtg_sensu Definition: Establishment of the specialized cytoplasm found at the poles of the egg. An example of this is found in Drosophila melanogaster. Relationships: is a type of cytoplasm organization [GO:0007028]; is a type of cellular component assembly [GO:0022607]; is part of oocyte anterior/posterior axis specification [GO:0007314]